{
  "gene_symbol": "GLYATL2",
  "gene": "UniProtKB:Q8WU03",
  "term_id": "UNKNOWN:0003",
  "gene_name": "Glycine N-acyltransferase-like protein 2",
  "term_label": "Unknown cellular component"
}